negative regulation of sterol biosynthetic process [GO:0106119] (biological process) References: PMID:16459310 Sources: GOC:BHF, GOC:BHF_miRNA, GOC:rph Relationships: is a type of negative regulation of steroid biosynthetic process [GO:0010894]; is a type of regulation of sterol biosynthetic process [GO:0106118]; RO_0002212 sterol biosynthetic process [GO:0016126] Subtypes: negative regulation of ergosterol biosynthetic process [GO:0010895], negative regulation of cholesterol biosynthetic process [GO:0045541] Definition: Any process that stops, prevents or reduces the frequency, rate or extent of a sterol biosynthetic process.